regulation of distal tip cell migration [GO:1903354] (biological process) Relationships: is a type of regulation of cell migration [GO:0030334]; regulates GO:0097628 Definition: Any process that modulates the frequency, rate or extent of distal tip cell migration. References: PMID:24968003 Sources: GOC:TermGenie, GOC:mm2, GO_REF:0000058 Subtypes: negative regulation of distal tip cell migration [GO:1903355], positive regulation of distal tip cell migration [GO:1903356]